{
  "term_label": "outer dynein arm assembly",
  "gene": "UniProtKB:Q4LDG9",
  "term_id": "GO:0036158",
  "gene_symbol": "DNAL1",
  "gene_name": "Dynein axonemal light chain 1"
}